{
  "gene_name": "Testis-specific Y-encoded-like protein 4",
  "term_label": "nucleus",
  "term_id": "GO:0005634",
  "gene": "UniProtKB:Q9UJ04",
  "gene_symbol": "TSPYL4"
}